{
  "term_label": "choline kinase activity",
  "term_id": "GO:0004103",
  "gene_name": "Choline_ethanolamine kinase",
  "gene": "UniProtKB:Q9Y259",
  "gene_symbol": "CHKB"
}